RNA polymerase I assembly [GO:1990113] (biological process) Also known as: DNA-directed RNA polymerase I complex assembly, RNA Polymerase I complex assembly Definition: The aggregation, arrangement and bonding together of a set of components to form the eukaryotic RNA polymerase I complex. References: PMID:23459708 Sources: GOC:rb Relationships: is a type of protein-containing complex assembly [GO:0065003]